{
  "gene_symbol": "DHX38",
  "gene": "UniProtKB:Q92620",
  "term_label": "spliceosomal complex",
  "gene_name": "Pre-mRNA-splicing factor ATP-dependent RNA helicase PRP16",
  "term_id": "GO:0005681"
}